GMP kinase activity [GO:0004385] (molecular function) Definition: Catalysis of the reaction: ATP + GMP = ADP + GDP. Sources: RHEA:20780 Also known as: membrane-associated guanylate kinase, 5'-GMP kinase activity, ATP:(d)GMP phosphotransferase activity, ATP:GMP phosphotransferase activity, deoxyguanylate kinase activity, guanosine monophosphate kinase activity, guanylate kinase activity Relationships: is a type of nucleoside monophosphate kinase activity [GO:0050145]; is part of GO:0046037; is part of GDP metabolic process [GO:0046710]